{
  "term_label": "endosome to lysosome transport",
  "gene_name": "Sorting nexin-16",
  "gene": "UniProtKB:P57768",
  "gene_symbol": "SNX16",
  "term_id": "GO:0008333"
}